{
  "term_label": "epidermal growth factor receptor signaling pathway",
  "gene_symbol": "BCAR3",
  "gene": "UniProtKB:O75815",
  "term_id": "GO:0007173",
  "gene_name": "Breast cancer anti-estrogen resistance protein 3"
}